{
  "term_label": "extracellular space",
  "term_id": "GO:0005615",
  "gene_symbol": "SMOC2",
  "gene": "UniProtKB:Q9H3U7",
  "gene_name": "SPARC-related modular calcium-binding protein 2"
}